{
  "gene": "UniProtKB:A7E2F4",
  "gene_name": "Golgin subfamily A member 8A",
  "gene_symbol": "GOLGA8A",
  "term_label": "Golgi cis cisterna",
  "term_id": "GO:0000137"
}